{
  "term_label": "ubiquitin protein ligase activity",
  "gene_name": "E3 ubiquitin-protein ligase DTX4",
  "gene_symbol": "DTX4",
  "gene": "UniProtKB:Q9Y2E6",
  "term_id": "GO:0061630"
}